{
  "gene_symbol": "ZNF10",
  "gene_name": "Zinc finger protein 10",
  "term_label": "nucleus",
  "term_id": "GO:0005634",
  "gene": "UniProtKB:P21506"
}